ascospore-type prospore membrane formation [GO:0032120] (biological process) Regulation: regulated by regulation of ascospore-type prospore membrane formation [GO:1903023]; positively regulated by positive regulation of ascospore-type prospore membrane formation [GO:1903024] Relationships: is a type of developmental process involved in reproduction [GO:0003006]; is a type of cellular component assembly involved in morphogenesis [GO:0010927]; is a type of membrane assembly [GO:0071709]; is a type of meiotic cell cycle process [GO:1903046]; is part of ascospore-type prospore assembly [GO:0031321] References: PMID:27630265 Sources: GOC:clt Also known as: FSM assembly, FSM biosynthesis, FSM formation, forespore membrane biosynthesis, forespore membrane formation, ascospore-type prospore membrane assembly, prospore membrane biogenesis Definition: The process in which the nascent membrane forms at the meiotic outer plaque and grows until closure occurs and forespores, or prospores, are formed.